estrone secretion [GO:0035943] (biological process) Definition: The regulated release of estrone into the circulatory system. Relationships: is a type of organic hydroxy compound transport [GO:0015850]; is a type of steroid hormone secretion [GO:0035929] Also known as: 3-hydroxy-1,3,5(10)-estratrien-17-one secretion, folliculin secretion References: PMID:8395854 Sources: GOC:sl Regulation: regulated by GO:2000867; negatively regulated by negative regulation of estrone secretion [GO:2000868]; positively regulated by positive regulation of estrone secretion [GO:2000869]